{
  "term_id": "GO:0042742",
  "term_label": "defense response to bacterium",
  "gene_name": "Dermcidin",
  "gene": "UniProtKB:P81605",
  "gene_symbol": "DCD"
}